{
  "term_label": "regulation of protein stability",
  "gene_name": "Ubl carboxyl-terminal hydrolase 18",
  "gene_symbol": "USP18",
  "gene": "UniProtKB:Q9UMW8",
  "term_id": "GO:0031647"
}